{
  "term_label": "promoter-specific chromatin binding",
  "gene_symbol": "PCGF2",
  "gene": "UniProtKB:P35227",
  "gene_name": "Polycomb group RING finger protein 2",
  "term_id": "GO:1990841"
}